{
  "term_id": "UNKNOWN:0003",
  "gene": "UniProtKB:Q96M89",
  "gene_name": "Coiled-coil domain-containing protein 138",
  "term_label": "Unknown cellular component",
  "gene_symbol": "CCDC138"
}